DNA strand elongation involved in mitotic DNA replication [GO:1902983] (BP) Also known as: DNA strand elongation involved in mitotic cell cycle DNA replication Sources: GOC:TermGenie, GO_REF:0000060 Relationships: is a type of DNA strand elongation involved in nuclear cell cycle DNA replication [GO:1902319]; is a type of GO:1903047; is part of mitotic DNA replication [GO:1902969] Definition: Any DNA strand elongation involved in mitotic cell cycle DNA replication. Subtypes: mitotic DNA replication lagging strand elongation [GO:1903459], mitotic DNA replication leading strand elongation [GO:1903460]